L-serine hydro-lyase (adding indole, L-tryptophan-forming) activity [GO:0052684] (molecular function) Sources: MetaCyc:RXN0-2382 Also known as: L-serine hydro-lyase (adding indole; L-tryptophan-forming) activity, tryptophan synthase beta subunit activity Relationships: is a type of GO:0016836 Definition: Catalysis of the reaction: indole + L-serine = L-tryptophan + H2O.